{
  "term_id": "GO:0060326",
  "gene_name": "Ras-related C3 botulinum toxin substrate 3",
  "gene_symbol": "RAC3",
  "gene": "UniProtKB:P60763",
  "term_label": "cell chemotaxis"
}